N4-acetylcytidine amidohydrolase activity [GO:0106251] (MF) References: PMID:31964920 Sources: GOC:imk, RHEA:62932 Relationships: is a type of hydrolase activity, acting on carbon-nitrogen (but not peptide) bonds, in linear amides [GO:0016811] Definition: Catalysis of the reaction N4-acetylcytidine +H2O = cytidine + acetate.